{
  "gene_name": "Calretinin",
  "term_id": "UNKNOWN:0002",
  "term_label": "Unknown biological process",
  "gene_symbol": "CALB2",
  "gene": "UniProtKB:P22676"
}